{
  "term_label": "sperm flagellum",
  "gene_name": "Sperm acrosome-associated protein 9",
  "gene": "UniProtKB:Q96E40",
  "term_id": "GO:0036126",
  "gene_symbol": "SPACA9"
}